negative regulation of gene expression, epigenetic [GO:0045814] (biological process) Also known as: down regulation of gene expression, epigenetic, down-regulation of gene expression, epigenetic, downregulation of gene expression, epigenetic, inhibition of gene expression, epigenetic, gene silencing References: PMID:22243696 Definition: An epigenetic process that silences gene expression at specific genomic regions through chromatin remodeling either by modifying higher order chromatin fiber structure, nucleosomal histones, or the cytosine DNA methylation. Subtypes: heterochromatin formation [GO:0031507], negative regulation of gene expression via chromosomal CpG island methylation [GO:0044027] Relationships: is a type of negative regulation of gene expression [GO:0010629]; is a type of GO:0040029